cellular response to nitrate [GO:0071249] (biological process) Sources: GOC:mah Definition: Any process that results in a change in state or activity of a cell (in terms of movement, secretion, enzyme production, gene expression, etc.) as a result of a nitrate stimulus. Relationships: is a type of response to nitrate [GO:0010167]; is a type of cellular response to oxygen-containing compound [GO:1901701]; is a type of GO:1902170